{
  "gene_name": "Plasma alpha-L-fucosidase",
  "term_label": "lysosome",
  "term_id": "GO:0005764",
  "gene": "UniProtKB:Q9BTY2",
  "gene_symbol": "FUCA2"
}